{
  "gene_symbol": "GABRG1",
  "term_label": "GABA-gated chloride ion channel activity",
  "term_id": "GO:0022851",
  "gene_name": "Gamma-aminobutyric acid receptor subunit gamma-1",
  "gene": "UniProtKB:Q8N1C3"
}